trans-Golgi network to recycling endosome transport [GO:0044795] (biological process) Relationships: is a type of endosomal transport [GO:0016197] References: PMID:18779367 Sources: GOC:lb Definition: The directed movement of substances, in membrane-bounded vesicles, from the trans-Golgi network to the recycling endosomes.